negative regulation of circadian sleep/wake cycle, non-REM sleep [GO:0042323] (BP) Definition: Any process that stops, prevents or reduces the duration or quality of non-rapid eye movement (NREM) sleep. Sources: GOC:jl Also known as: down regulation of circadian sleep/wake cycle, non-REM sleep, down-regulation of circadian sleep/wake cycle, non-REM sleep, downregulation of circadian sleep/wake cycle, non-REM sleep, negative regulation of non-REM sleep, inhibition of circadian sleep/wake cycle, non-REM sleep Relationships: is a type of negative regulation of circadian sleep/wake cycle, sleep [GO:0042321]; is a type of GO:0045188; negatively regulates circadian sleep/wake cycle, non-REM sleep [GO:0042748]